{
  "gene_name": "E3 ubiquitin-protein ligase MSL2",
  "gene": "UniProtKB:Q9HCI7",
  "term_id": "GO:0016567",
  "gene_symbol": "MSL2",
  "term_label": "protein ubiquitination"
}